{
  "term_label": "Unknown molecular function",
  "gene_symbol": "SAP130",
  "term_id": "UNKNOWN:0001",
  "gene": "UniProtKB:Q9H0E3",
  "gene_name": "Histone deacetylase complex subunit SAP130"
}